{
  "gene_symbol": "TNFSF4",
  "gene": "UniProtKB:P23510",
  "gene_name": "Tumor necrosis factor ligand superfamily member 4",
  "term_id": "GO:0001819",
  "term_label": "positive regulation of cytokine production"
}